{
  "term_id": "UNKNOWN:0001",
  "gene": "UniProtKB:Q9UGK8",
  "term_label": "Unknown molecular function",
  "gene_symbol": "SERGEF",
  "gene_name": "Secretion-regulating guanine nucleotide exchange factor"
}